polyvinyl alcohol dehydrogenase (cytochrome) activity [GO:0047059] (MF) Also known as: PVA dehydrogenase activity, polyvinyl-alcohol:(acceptor) oxidoreductase activity, polyvinyl-alcohol:acceptor oxidoreductase activity, polyvinyl alcohol:ferricytochrome-c oxidoreductase activity Definition: Catalysis of the reaction: polyvinyl alcohol + ferricytochrome c = oxidized polyvinyl alcohol + ferrocytochrome c + H+. Sources: EC:1.1.2.6 Relationships: is_a oxidoreductase activity, acting on the CH-OH group of donors, cytochrome as acceptor [GO:0016898]